{
  "gene_symbol": "TRMT10C",
  "gene_name": "tRNA methyltransferase 10 homolog C",
  "term_label": "positive regulation of mitochondrial translation",
  "term_id": "GO:0070131",
  "gene": "UniProtKB:Q7L0Y3"
}